glutathione gamma-glutamylcysteinyltransferase activity [GO:0016756] (molecular function) Relationships: is a type of aminoacyltransferase activity [GO:0016755] Also known as: phytochelatin synthase activity Sources: EC:2.3.2.15 Definition: Catalysis of the reaction: glutathione + Glu(-Cys)(n)-Gly = Gly + Glu(-Cys)(n+1)-Gly.